{
  "term_label": "small GTPase-mediated signal transduction",
  "term_id": "GO:0007264",
  "gene_name": "GTP-binding protein Rheb",
  "gene_symbol": "RHEB",
  "gene": "UniProtKB:Q15382"
}